regulation of optical nerve axon regeneration [GO:1905591] (biological process) Relationships: is a type of regulation of axon regeneration [GO:0048679]; RO_0002211 optical nerve axon regeneration [GO:0101027] Definition: Any process that modulates the frequency, rate or extent of optical nerve axon regeneration. References: PMID:16699509 Sources: GOC:TermGenie, GO_REF:0000058 Subtypes: negative regulation of optical nerve axon regeneration [GO:1905592], positive regulation of optical nerve axon regeneration [GO:1905593]